negative regulation of acinar cell proliferation [GO:1904698] (biological process) Definition: Any process that stops, prevents or reduces the frequency, rate or extent of acinar cell proliferation. References: PMID:9788538 Sources: GOC:TermGenie, GO_REF:0000058 Also known as: down regulation of acinar cell proliferation, down regulation of acinic cell proliferation, down regulation of acinous cell proliferation, down-regulation of acinar cell proliferation, down-regulation of acinic cell proliferation, down-regulation of acinous cell proliferation, downregulation of acinar cell proliferation, downregulation of acinic cell proliferation, downregulation of acinous cell proliferation, negative regulation of acinic cell proliferation, negative regulation of acinous cell proliferation, inhibition of acinar cell proliferation, inhibition of acinic cell proliferation, inhibition of acinous cell proliferation Relationships: is a type of negative regulation of epithelial cell proliferation [GO:0050680]; is a type of GO:1904697; negatively regulates acinar cell proliferation [GO:1990863]